protein phosphatase regulator activity [GO:0019888] (MF) Relationships: is a type of phosphatase regulator activity [GO:0019208]; has part protein phosphatase binding [GO:0019903]; regulates GO:0004721 Sources: GOC:ai Definition: Binds to and modulates the activity of a protein phosphatase. Subtypes: protein phosphatase inhibitor activity [GO:0004864], GO:0008597, GO:0017020, protein phosphatase activator activity [GO:0072542] Also known as: calcineurin regulator activity, calcineurin, intrinsic regulator activity, protein phosphatase 2 regulator activity, protein phosphatase 2, intrinsic regulator activity, protein phosphatase 3 regulator activity, protein phosphatase 3, intrinsic regulator activity, protein phosphatase type 1 regulator activity, protein phosphatase type 1, intrinsic regulator activity, protein phosphatase type 2A regulator activity, protein phosphatase type 2A, intrinsic regulator activity, protein phosphatase type 2B regulator activity, protein phosphatase type 2B, intrinsic regulator activity, protein phosphatase type 4 regulator activity, protein phosphatase type 4, intrinsic regulator activity